{
  "gene_symbol": "CD200",
  "gene_name": "OX-2 membrane glycoprotein",
  "term_id": "GO:0098632",
  "term_label": "cell-cell adhesion mediator activity",
  "gene": "UniProtKB:P41217"
}